{
  "gene": "UniProtKB:Q7Z2E3",
  "term_label": "single strand break repair",
  "gene_symbol": "APTX",
  "gene_name": "Aprataxin",
  "term_id": "GO:0000012"
}